{
  "gene": "UniProtKB:Q13822",
  "gene_symbol": "ENPP2",
  "gene_name": "Ectonucleotide pyrophosphatase_phosphodiesterase family member 2",
  "term_label": "phosphatidylcholine catabolic process",
  "term_id": "GO:0034638"
}